{
  "gene": "UniProtKB:Q9H3M9",
  "term_id": "GO:0005634",
  "gene_name": "Ataxin-3-like protein",
  "term_label": "nucleus",
  "gene_symbol": "ATXN3L"
}